{
  "gene_symbol": "ZNF45",
  "gene": "UniProtKB:Q02386",
  "term_id": "UNKNOWN:0001",
  "gene_name": "Zinc finger protein 45",
  "term_label": "Unknown molecular function"
}